{
  "term_label": "protein ubiquitination",
  "term_id": "GO:0016567",
  "gene_symbol": "RPGR",
  "gene_name": "X-linked retinitis pigmentosa GTPase regulator",
  "gene": "UniProtKB:Q92834"
}